{
  "gene": "UniProtKB:P15529",
  "gene_name": "Membrane cofactor protein",
  "gene_symbol": "CD46",
  "term_id": "UNKNOWN:0001",
  "term_label": "Unknown molecular function"
}